regulation of receptor-mediated endocytosis involved in cholesterol transport [GO:1905600] (biological process) Subtypes: GO:1905601, GO:1905602 Definition: Any process that modulates the frequency, rate or extent of receptor-mediated endocytosis involved in cholesterol transport. Relationships: is_a GO:0032386; is_a regulation of receptor-mediated endocytosis [GO:0048259]; regulates GO:0090118 Also known as: regulation of receptor-mediated endocytosis involved in intracellular cholesterol transport, regulation of receptor-mediated endocytosis of LDL, regulation of receptor-mediated endocytosis of low-density lipoprotein involved in cholesterol transport, regulation of receptor-mediated endocytosis of low-density lipoprotein particle involved in cholesterol transport References: PMID:22848640 Sources: GOC:BHF, GOC:TermGenie, GOC:nc, GO_REF:0000058